{
  "term_label": "midbody",
  "gene_symbol": "ALKBH4",
  "gene_name": "Alpha-ketoglutarate-dependent dioxygenase alkB homolog 4",
  "term_id": "GO:0030496",
  "gene": "UniProtKB:Q9NXW9"
}